{
  "gene_name": "Superoxide dismutase [Cu-Zn]",
  "gene_symbol": "SOD1",
  "term_label": "superoxide dismutase activity",
  "gene": "UniProtKB:P00441",
  "term_id": "GO:0004784"
}